{
  "term_id": "GO:0045840",
  "gene_name": "Protransforming growth factor alpha",
  "gene_symbol": "TGFA",
  "term_label": "positive regulation of mitotic nuclear division",
  "gene": "UniProtKB:P01135"
}